monoatomic cation transport [GO:0006812] (biological process) Definition: The directed movement of a monoatomic cation, into, out of or within a cell, or between cells, by means of some agent such as a transporter or pore. Monatomic cations (also called simple cations) are positively charged ions consisting of exactly one atom. Sources: GOC:ai Subtypes: metal ion transport [GO:0030001], monoatomic cation transmembrane transport [GO:0098655] Also known as: cation transport, di-, tri-valent inorganic cation transport, trivalent inorganic cation transport Relationships: is a type of monoatomic ion transport [GO:0006811]